{
  "gene_symbol": "HABP4",
  "term_id": "GO:0045948",
  "gene": "UniProtKB:Q5JVS0",
  "gene_name": "Intracellular hyaluronan-binding protein 4",
  "term_label": "positive regulation of translational initiation"
}